methylamine dehydrogenase (amicyanin) activity [GO:0052876] (molecular function) Definition: Catalysis of the reaction: 2O + methylamine + 2 oxidized [amicyanin] = formaldehyde + 2 H+ + NH4+ + 2 reduced [amicyanin]. Sources: RHEA:30207 Relationships: is a type of oxidoreductase activity, acting on the CH-NH2 group of donors, with a copper protein as acceptor [GO:0052877] Also known as: MADH activity, amine dehydrogenase, primary-amine dehydrogenase, methylamine dehydrogenase activity, methylamine:amicyanin oxidoreductase (deaminating) activity